{
  "gene": "UniProtKB:Q9Y6D0",
  "gene_name": "Selenoprotein K",
  "term_label": "Golgi apparatus",
  "gene_symbol": "SELENOK",
  "term_id": "GO:0005794"
}